positive regulation of intracellular cholesterol transport [GO:0032385] (biological process) Definition: Any process that activates or increases the frequency, rate or extent of the directed movement of cholesterol within cells. Also known as: up regulation of intracellular cholesterol transport, up-regulation of intracellular cholesterol transport, upregulation of intracellular cholesterol transport, activation of intracellular cholesterol transport, stimulation of intracellular cholesterol transport Relationships: is a type of positive regulation of cholesterol transport [GO:0032376]; is a type of positive regulation of intracellular sterol transport [GO:0032382]; is a type of regulation of intracellular cholesterol transport [GO:0032383]; RO_0002213 intracellular cholesterol transport [GO:0032367] Sources: GOC:mah Subtypes: positive regulation of receptor-mediated endocytosis involved in cholesterol transport [GO:1905602]